{
  "term_label": "extracellular space",
  "gene_name": "Angiopoietin-related protein 3",
  "gene": "UniProtKB:Q9Y5C1",
  "gene_symbol": "ANGPTL3",
  "term_id": "GO:0005615"
}